{
  "gene_symbol": "CLEC4C",
  "term_label": "pattern recognition receptor activity",
  "term_id": "GO:0038187",
  "gene": "UniProtKB:Q8WTT0",
  "gene_name": "C-type lectin domain family 4 member C"
}